{
  "term_id": "GO:0005886",
  "term_label": "plasma membrane",
  "gene_name": "Transmembrane protein 202",
  "gene": "UniProtKB:A6NGA9",
  "gene_symbol": "TMEM202"
}